{
  "gene_symbol": "ACACA",
  "term_label": "acetyl-CoA carboxylase activity",
  "term_id": "GO:0003989",
  "gene": "UniProtKB:Q13085",
  "gene_name": "Acetyl-CoA carboxylase 1"
}